{
  "gene_name": "ETS translocation variant 5",
  "term_label": "regulation of transcription by RNA polymerase II",
  "gene": "UniProtKB:P41161",
  "term_id": "GO:0006357",
  "gene_symbol": "ETV5"
}